{
  "term_id": "UNKNOWN:0002",
  "term_label": "Unknown biological process",
  "gene_symbol": "AMMECR1",
  "gene": "UniProtKB:Q9Y4X0",
  "gene_name": "Nuclear protein AMMECR1"
}